positive regulation of B cell apoptotic process [GO:0002904] (biological process) Relationships: is a type of GO:0002902; is a type of GO:0070230; positively regulates B cell apoptotic process [GO:0001783] Also known as: up regulation of B cell apoptosis, up-regulation of B cell apoptosis, upregulation of B cell apoptosis, activation of B cell apoptosis, positive regulation of B cell apoptosis, stimulation of B cell apoptosis Sources: GOC:add, GOC:mtg_apoptosis Subtypes: GO:0002869, positive regulation of mature B cell apoptotic process [GO:0002907] Definition: Any process that activates or increases the frequency, rate, or extent of B cell apoptotic process.